{
  "term_id": "UNKNOWN:0003",
  "gene_symbol": "E4F1",
  "gene": "UniProtKB:Q66K89",
  "term_label": "Unknown cellular component",
  "gene_name": "Transcription factor E4F1"
}